exopher [GO:0160014] (CC) References: PMID:28178240, PMID:33016946, PMID:33027673, PMID:33659873, PMID:34288362, PMID:34475208 Definition: An extracellular vesicle that is approximately four microns in diameter, released by budding out of cells into the extracellular space, and hypothesized to be a mechanism for disposal of unwanted cellular material including protein aggregates and damaged organelles. Relationships: is a type of extracellular vesicle [GO:1903561]